{
  "term_label": "spermatogenesis",
  "gene_name": "Tudor domain-containing protein 6",
  "gene_symbol": "TDRD6",
  "gene": "UniProtKB:O60522",
  "term_id": "GO:0007283"
}